{
  "gene": "UniProtKB:O15467",
  "gene_symbol": "CCL16",
  "term_label": "extracellular space",
  "gene_name": "C-C motif chemokine 16",
  "term_id": "GO:0005615"
}